{
  "term_label": "epithelial cell differentiation",
  "gene_symbol": "KRT38",
  "term_id": "GO:0030855",
  "gene": "UniProtKB:O76015",
  "gene_name": "Keratin, type I cuticular Ha8"
}